tail-anchored membrane protein insertion into ER membrane [GO:0071816] (biological process) Definition: A process of protein insertion into the endoplasmic reticulum (ER) membrane in which a tail-anchored (TA) transmembrane protein is incorporated into an endoplasmic reticulum (ER) membrane. TA transmembrane protein, also named type II transmembrane proteins, contain a single C- terminal transmembrane region. References: PMID:20516149, PMID:20676083 Sources: GOC:mah, GOC:sp Also known as: protein insertion of tail-anchored membrane proteins into ER membrane, tail-anchored membrane protein insertion into endoplasmic reticulum membrane, type II transmembrane protein insertion into ER membrane Relationships: is a type of protein insertion into ER membrane [GO:0045048]